3,4-dihydroxyphenylacetate 2,3-dioxygenase activity [GO:0008687] (molecular function) Definition: Catalysis of the reaction: 3,4-dihydroxyphenylacetate + O2 = 5-formyl-2-hydroxyhepta-2,4-dienedioate + H+. Sources: RHEA:15633 Also known as: 3,4-dihydroxyphenylacetate:oxygen 2,3-oxidoreductase (decyclizing), 3,4-dihydroxyphenylacetic acid 2,3-dioxygenase activity, HPC dioxygenase activity, homoprotocatechuate 2,3-dioxygenase activity Relationships: is a type of GO:0016702